{
  "term_id": "UNKNOWN:0003",
  "gene_symbol": "FBXW5",
  "gene": "UniProtKB:Q969U6",
  "term_label": "Unknown cellular component",
  "gene_name": "F-box_WD repeat-containing protein 5"
}